{
  "term_id": "GO:0008783",
  "gene_name": "Guanidino acid hydrolase, mitochondrial",
  "term_label": "agmatinase activity",
  "gene": "UniProtKB:Q9BSE5",
  "gene_symbol": "AGMAT"
}